{
  "term_id": "UNKNOWN:0003",
  "term_label": "Unknown cellular component",
  "gene_name": "Purkinje cell protein 2 homolog",
  "gene": "UniProtKB:Q8IVA1",
  "gene_symbol": "PCP2"
}